response to clozapine [GO:0097338] (biological process) Definition: Any process that results in a change in state or activity of a cell or an organism (in terms of movement, secretion, enzyme production, gene expression, etc.) as a result of a clozapine stimulus. Sources: GOC:pr Relationships: is a type of response to nitrogen compound [GO:1901698]